{
  "gene_name": "UBX domain-containing protein 2B",
  "gene": "UniProtKB:Q14CS0",
  "gene_symbol": "UBXN2B",
  "term_id": "GO:0000045",
  "term_label": "autophagosome assembly"
}